{
  "term_id": "UNKNOWN:0001",
  "gene_name": "Peptidyl-prolyl cis-trans isomerase FKBP3",
  "gene": "UniProtKB:Q00688",
  "gene_symbol": "FKBP3",
  "term_label": "Unknown molecular function"
}